methionine import across plasma membrane [GO:1903692] (biological process) References: PMID:17556368 Sources: GOC:TermGenie, GO_REF:0000075 Also known as: methionine import, methionine import into cell Relationships: is a type of methionine transport [GO:0015821]; is a type of amino acid import across plasma membrane [GO:0089718]; is a type of carboxylic acid transmembrane transport [GO:1905039] Subtypes: L-methionine import across plasma membrane [GO:1905544] Definition: The directed movement of methionine from outside of a cell, across the plasma membrane and into the cytosol.